{
  "gene": "UniProtKB:P0C851",
  "gene_name": "Phosphoinositide-interacting protein",
  "gene_symbol": "PIRT",
  "term_id": "GO:1902936",
  "term_label": "phosphatidylinositol bisphosphate binding"
}